{
  "term_label": "axoneme",
  "gene": "UniProtKB:Q9P0W8",
  "gene_symbol": "SPATA7",
  "term_id": "GO:0005930",
  "gene_name": "Spermatogenesis-associated protein 7"
}